{
  "gene": "UniProtKB:O60894",
  "term_id": "GO:0015031",
  "gene_name": "Receptor activity-modifying protein 1",
  "gene_symbol": "RAMP1",
  "term_label": "protein transport"
}